{
  "gene": "UniProtKB:Q9H930",
  "gene_name": "Nuclear body protein SP140-like protein",
  "term_id": "GO:0000981",
  "gene_symbol": "SP140L",
  "term_label": "DNA-binding transcription factor activity, RNA polymerase II-specific"
}